{
  "term_id": "GO:0043409",
  "term_label": "negative regulation of MAPK cascade",
  "gene_symbol": "DUSP29",
  "gene": "UniProtKB:Q68J44",
  "gene_name": "Dual specificity phosphatase 29"
}